{
  "gene": "UniProtKB:P12235",
  "term_label": "regulation of mitochondrial membrane permeability",
  "gene_symbol": "SLC25A4",
  "term_id": "GO:0046902",
  "gene_name": "ADP_ATP translocase 1"
}